{
  "gene_name": "Potassium-transporting ATPase subunit beta",
  "term_label": "intracellular sodium ion homeostasis",
  "term_id": "GO:0006883",
  "gene": "UniProtKB:P51164",
  "gene_symbol": "ATP4B"
}